{
  "gene_name": "Choline transporter-like protein 3",
  "gene": "UniProtKB:Q8N4M1",
  "gene_symbol": "SLC44A3",
  "term_label": "transmembrane transport",
  "term_id": "GO:0055085"
}